{
  "gene": "UniProtKB:Q9H8W4",
  "gene_name": "Pleckstrin homology domain-containing family F member 2",
  "gene_symbol": "PLEKHF2",
  "term_label": "phosphatidylinositol binding",
  "term_id": "GO:0035091"
}